{
  "term_label": "regulation of transcription by RNA polymerase II",
  "gene": "UniProtKB:Q3ZCT1",
  "gene_symbol": "ZNF260",
  "term_id": "GO:0006357",
  "gene_name": "Zinc finger protein 260"
}